{
  "term_id": "UNKNOWN:0001",
  "term_label": "Unknown molecular function",
  "gene_symbol": "YIF1A",
  "gene_name": "Protein YIF1A",
  "gene": "UniProtKB:O95070"
}